butyryl-CoA catabolic process to butanol [GO:0044582] (biological process) Regulation: regulated by GO:1900497; negatively regulated by negative regulation of butyryl-CoA catabolic process to butanol [GO:1900498]; positively regulated by GO:1900499 References: PMID:19539744 Sources: GOC:mengo_curators, GOC:tt Also known as: butyryl-CoA catabolism to butanol Definition: The chemical reactions a resulting in the resulting in the breakdown of butyryl-CoA to form butanol. Relationships: is a type of GO:0044580; is a type of GO:0071271